{
  "gene_symbol": "SMARCA5",
  "term_id": "GO:0003677",
  "term_label": "DNA binding",
  "gene_name": "SWI_SNF-related matrix-associated actin-dependent regulator of chromatin subfamily A member 5",
  "gene": "UniProtKB:O60264"
}